{
  "gene_name": "Atos homolog protein A",
  "term_label": "Unknown cellular component",
  "term_id": "UNKNOWN:0003",
  "gene_symbol": "ATOSA",
  "gene": "UniProtKB:Q32MH5"
}